guanidinodeoxy-scyllo-inositol-4-phosphatase activity [GO:0047383] (molecular function) Definition: Catalysis of the reaction: 1-guanidino-1-deoxy-scyllo-inositol 4-phosphate + H2O = 1-guanidino-1-deoxy-scyllo-inositol + phosphate. Sources: EC:3.1.3.40, RHEA:15777 Also known as: 1-guanidino-1-deoxy-scyllo-inositol-4-P phosphohydrolase activity, 1-guanidino-1-deoxy-scyllo-inositol-4-phosphate 4-phosphohydrolase activity, 1-guanidino-scyllo-inositol 4-phosphatase activity Relationships: is a type of GO:0016791